{
  "gene_name": "Uncharacterized protein C14orf178",
  "gene_symbol": "C14orf178",
  "gene": "UniProtKB:Q8N769",
  "term_id": "UNKNOWN:0003",
  "term_label": "Unknown cellular component"
}